{
  "term_id": "GO:0005886",
  "gene_name": "Fibronectin type III domain-containing protein 5",
  "gene_symbol": "FNDC5",
  "gene": "UniProtKB:Q8NAU1",
  "term_label": "plasma membrane"
}